{
  "term_label": "protein-lysine N-methyltransferase activity",
  "gene": "UniProtKB:P0DPD7",
  "term_id": "GO:0016279",
  "gene_symbol": "EEF1AKMT4",
  "gene_name": "EEF1A lysine methyltransferase 4"
}